{
  "term_id": "GO:0034625",
  "term_label": "fatty acid elongation, monounsaturated fatty acid",
  "gene_name": "Elongation of very long chain fatty acids protein 2",
  "gene_symbol": "ELOVL2",
  "gene": "UniProtKB:Q9NXB9"
}